{
  "gene_name": "Tripartite motif-containing protein 3",
  "term_id": "GO:0061630",
  "term_label": "ubiquitin protein ligase activity",
  "gene": "UniProtKB:O75382",
  "gene_symbol": "TRIM3"
}